{
  "term_id": "GO:0005886",
  "term_label": "plasma membrane",
  "gene_symbol": "ABCG4",
  "gene": "UniProtKB:Q9H172",
  "gene_name": "ATP-binding cassette sub-family G member 4"
}